{
  "gene_symbol": "OR6C70",
  "gene_name": "Olfactory receptor 6C70",
  "gene": "UniProtKB:A6NIJ9",
  "term_id": "UNKNOWN:0002",
  "term_label": "Unknown biological process"
}